methylgallate catabolic process [GO:0046276] (biological process) Definition: The chemical reactions and pathways resulting in the breakdown of methylgallate, trihydroxymethylbenzoate, the anion of methylgallic acid. Relationships: is a type of catechol-containing compound catabolic process [GO:0019614]; is a type of benzene-containing compound metabolic process [GO:0042537]; is a type of monocarboxylic acid catabolic process [GO:0072329] Also known as: methylgallate breakdown, methylgallate catabolism, methylgallate degradation Sources: GOC:ai